{
  "term_id": "GO:0005741",
  "term_label": "mitochondrial outer membrane",
  "gene_name": "CDGSH iron-sulfur domain-containing protein 1",
  "gene": "UniProtKB:Q9NZ45",
  "gene_symbol": "CISD1"
}